{
  "gene_name": "Nuclear RNA export factor 3",
  "term_label": "poly(A)+ mRNA export from nucleus",
  "gene_symbol": "NXF3",
  "term_id": "GO:0016973",
  "gene": "UniProtKB:Q9H4D5"
}